purine nucleotide-sugar transmembrane transport [GO:0090480] (biological process) Relationships: is a type of nucleotide-sugar transmembrane transport [GO:0015780] Sources: GOC:tb Note: Note that this term is not intended for use in annotating lateral movement within membranes. Also known as: purine nucleotide-sugar membrane transport, purine nucleotide-sugar transport Subtypes: GO:0015783, GO:1990570 Definition: The process in which a purine nucleotide-sugar is transported across a membrane. Purine nucleotide-sugars are purine nucleotides in glycosidic linkage with a monosaccharide or monosaccharide derivative.